{
  "gene_name": "Deoxyribonuclease-1-like 2",
  "gene": "UniProtKB:Q92874",
  "term_label": "DNA binding",
  "gene_symbol": "DNASE1L2",
  "term_id": "GO:0003677"
}